{
  "gene_name": "Protein BEX5",
  "term_label": "signal transduction",
  "gene": "UniProtKB:Q5H9J7",
  "term_id": "GO:0007165",
  "gene_symbol": "BEX5"
}